autosome genomic imprinting [GO:0141068] (biological process) Definition: The establishment of epigenetic modifications (imprints) in autosomal (non-sexual) chromosomes during gametogenesis, and propagation of these imprints during the organism's life. Genomic imprinting leads to an asymmetry between the maternal and paternal alleles and differential expression of the corresponding alleles. This can happen through heterochromatin formation or differential chromatin loop formation. References: PMID:31782494 Relationships: is a type of genomic imprinting [GO:0071514] Also known as: autosomal genomic imprinting, genomic imprinting of autosomal genes